{
  "gene_symbol": "TAS2R3",
  "term_id": "GO:0033038",
  "gene_name": "Taste receptor type 2 member 3",
  "term_label": "bitter taste receptor activity",
  "gene": "UniProtKB:Q9NYW6"
}